protein geranylgeranylation [GO:0018344] (biological process) Definition: The covalent attachment of a geranylgeranyl group to a protein. Sources: GOC:jl Also known as: protein amino acid geranylgeranylation, C-terminal protein geranylgeranylation Relationships: is a type of GO:0018342 Regulation: regulated by regulation of protein geranylgeranylation [GO:2000539]; negatively regulated by negative regulation of protein geranylgeranylation [GO:2000540]; RO_0002213 by positive regulation of protein geranylgeranylation [GO:2000541]